positive regulation of nutrient release by host [GO:0052092] (biological process) Definition: Any process in which an organism activates, maintains or increases the frequency, rate or extent of the release of nutrients from its host organism. The host is defined as the larger of the organisms involved in a symbiotic interaction. Relationships: is a type of modulation of nutrient release by host [GO:0052091] Also known as: positive regulation by symbiont of nutrient release from host, promotion of nutrient release from host, up regulation by symbiont of nutrient release from host, up-regulation by symbiont of nutrient release from host, upregulation by symbiont of nutrient release from host, activation by symbiont of nutrient release from host, stimulation by symbiont of nutrient release from host Sources: GOC:mtg_pamgo_17jul06